regulation of establishment or maintenance of bipolar cell polarity [GO:2000099] (biological process) Definition: Any process that modulates the frequency, rate or extent of establishment or maintenance of bipolar cell polarity. Sources: GOC:obol Relationships: is a type of GO:0032878; regulates GO:0061245 Subtypes: regulation of establishment or maintenance of bipolar cell polarity regulating cell shape [GO:2000100]